negative regulation of antigen processing and presentation of endogenous peptide antigen via MHC class I [GO:1904283] (biological process) Definition: Any process that stops, prevents or reduces the frequency, rate or extent of antigen processing and presentation of endogenous peptide antigen via MHC class I. Also known as: down regulation of antigen processing and presentation of endogenous peptide antigen via MHC class I, down regulation of endogenous peptide antigen processing and presentation via MHC class I, down-regulation of antigen processing and presentation of endogenous peptide antigen via MHC class I, down-regulation of endogenous peptide antigen processing and presentation via MHC class I, downregulation of antigen processing and presentation of endogenous peptide antigen via MHC class I, downregulation of endogenous peptide antigen processing and presentation via MHC class I, negative regulation of endogenous peptide antigen processing and presentation via MHC class I, inhibition of antigen processing and presentation of endogenous peptide antigen via MHC class I, inhibition of endogenous peptide antigen processing and presentation via MHC class I References: PMID:24643698 Sources: GOC:BHF, GOC:TermGenie, GOC:rl, GO_REF:0000058 Relationships: is a type of negative regulation of antigen processing and presentation of peptide antigen via MHC class I [GO:0002590]; is a type of regulation of antigen processing and presentation of endogenous peptide antigen via MHC class I [GO:1904282]; negatively regulates antigen processing and presentation of endogenous peptide antigen via MHC class I [GO:0019885]